{
  "gene": "UniProtKB:Q13232",
  "term_id": "UNKNOWN:0003",
  "gene_symbol": "NME3",
  "term_label": "Unknown cellular component",
  "gene_name": "Nucleoside diphosphate kinase 3"
}